{
  "term_id": "GO:0006888",
  "gene": "UniProtKB:O14579",
  "term_label": "endoplasmic reticulum to Golgi vesicle-mediated transport",
  "gene_symbol": "COPE",
  "gene_name": "Coatomer subunit epsilon"
}